{
  "gene_name": "Protein S100-A9",
  "term_id": "GO:0005509",
  "gene": "UniProtKB:P06702",
  "term_label": "calcium ion binding",
  "gene_symbol": "S100A9"
}